ciliary transition zone assembly [GO:1905349] (BP) References: PMID:21725307, PMID:23644468, PMID:24448408, PMID:26595381, PMID:26982032 Sources: GOC:TermGenie, GOC:cilia, GO_REF:0000079 Definition: The aggregation, arrangement and bonding together of a set of components to form a ciliary transition zone. Relationships: is a type of cellular component assembly [GO:0022607]; is part of cilium assembly [GO:0060271] Also known as: cilial transition zone assembly, cilial transition zone formation, ciliary transition zone formation, cilium transition zone assembly, cilium transition zone formation